response to interleukin-18 [GO:0070673] (biological process) Definition: Any process that results in a change in state or activity of a cell or an organism (in terms of movement, secretion, enzyme production, gene expression, etc.) as a result of an interleukin-18 stimulus. Relationships: is a type of response to cytokine [GO:0034097] Sources: GOC:mah Also known as: response to IL-18 Subtypes: cellular response to interleukin-18 [GO:0071351]